{
  "gene_name": "SH2 domain-containing adapter protein F",
  "gene": "UniProtKB:Q7M4L6",
  "term_label": "phosphotyrosine residue binding",
  "gene_symbol": "SHF",
  "term_id": "GO:0001784"
}